{
  "gene_symbol": "FUOM",
  "gene": "UniProtKB:A2VDF0",
  "gene_name": "Fucose mutarotase",
  "term_id": "GO:0016857",
  "term_label": "racemase and epimerase activity, acting on carbohydrates and derivatives"
}